{
  "gene_symbol": "RASSF7",
  "term_id": "UNKNOWN:0003",
  "term_label": "Unknown cellular component",
  "gene": "UniProtKB:Q02833",
  "gene_name": "Ras association domain-containing protein 7"
}